{
  "term_id": "UNKNOWN:0002",
  "gene_symbol": "CLEC18B",
  "gene_name": "C-type lectin domain family 18 member B",
  "term_label": "Unknown biological process",
  "gene": "UniProtKB:Q6UXF7"
}